{
  "gene_symbol": "TTYH2",
  "gene": "UniProtKB:Q9BSA4",
  "gene_name": "Protein tweety homolog 2",
  "term_id": "GO:0005229",
  "term_label": "intracellularly calcium-gated chloride channel activity"
}